negative regulation of tumor necrosis factor production [GO:0032720] (biological process) References: PMID:10891884, PMID:15560120 Sources: GOC:mah Relationships: is a type of regulation of tumor necrosis factor production [GO:0032680]; is a type of negative regulation of tumor necrosis factor superfamily cytokine production [GO:1903556]; negatively regulates GO:0032640 Also known as: down regulation of tumor necrosis factor production, down-regulation of tumor necrosis factor production, downregulation of tumor necrosis factor production, negative regulation TNF production, negative regulation TNF-alpha production, negative regulation tumor necrosis factor-alpha production, inhibition of cachectin production, inhibition of tumor necrosis factor production, negative regulation of tumor necrosis factor biosynthetic process, negative regulation of tumor necrosis factor secretion Definition: Any process that stops, prevents, or reduces the frequency, rate, or extent of tumor necrosis factor production. Note: Note that this term refers only to the specific, original 'tumor necrosis factor' protein (TNF) and not other members of the tumor necrosis factor superfamily (those with the gene symbol root 'TNFSF').